acetyl-CoA:CoA antiporter activity [GO:0015325] (molecular function) Relationships: is a type of acetyl-CoA transmembrane transporter activity [GO:0008521]; is a type of coenzyme A transmembrane transporter activity [GO:0015228]; is a type of antiporter activity [GO:0015297] Sources: TC:2.A.1.25.1 Definition: Catalysis of the reaction: acetyl-CoA(out) + CoA(in) = acetyl-CoA(in) + CoA(out).